{
  "term_id": "UNKNOWN:0001",
  "gene_symbol": "FAM90A13P",
  "gene": "UniProtKB:P0C7W8",
  "term_label": "Unknown molecular function",
  "gene_name": "Putative protein FAM90A13P"
}